folic acid biosynthetic process [GO:0046656] (biological process) Also known as: folate biosynthesis, folate biosynthetic process, folic acid anabolism, folic acid biosynthesis, folic acid formation, folic acid synthesis, vitamin B9 biosynthesis, vitamin B9 biosynthetic process, vitamin M biosynthesis, vitamin M biosynthetic process Sources: GOC:ai Relationships: is a type of folic acid-containing compound biosynthetic process [GO:0009396]; is a type of water-soluble vitamin biosynthetic process [GO:0042364]; is_a amide biosynthetic process [GO:0043604]; is a type of dicarboxylic acid biosynthetic process [GO:0043650]; is a type of GO:0046655 Definition: The chemical reactions and pathways resulting in the formation of folic acid, pteroylglutamic acid.